{
  "gene_symbol": "EHD1",
  "term_id": "GO:0060271",
  "gene_name": "EH domain-containing protein 1",
  "term_label": "cilium assembly",
  "gene": "UniProtKB:Q9H4M9"
}